lactaldehyde dehydrogenase (NAD+) activity [GO:0008911] (MF) Also known as: (S)-lactaldehyde:NAD+ oxidoreductase activity, L-lactaldehyde:NAD oxidoreductase activity, nicotinamide adenine dinucleotide (NAD)-linked dehydrogenase activity Definition: Catalysis of the reaction: (S)-lactaldehyde + NAD+ + H2O = (S)-lactate + NADH + H+. Relationships: is a type of aldehyde dehydrogenase (NAD+) activity [GO:0004029] Sources: RHEA:14277